CORVET complex [GO:0033263] (cellular component) Relationships: is a type of vesicle tethering complex [GO:0099023]; BFO_0000050 GO:0005768 References: PMID:17488625 Definition: A multimeric protein complex that acts as an endosomal tethering complex (CORVET = class C core vacuole/endosome tethering) by cooperating with Rab GTPases to capture endosomal vesicles and trap them prior to the action of SNAREs; the complex is involved in endo-lysosomal biogenesis and required for transport between endosome and vacuole. The Saccharomyces cerevisiae complex contains Vps8p, Vps3p, Pep5p, Vps16p, Pep3p, and Vps33p.